{
  "gene": "UniProtKB:Q9BZQ2",
  "gene_symbol": "SHCBP1L",
  "term_id": "GO:0007112",
  "term_label": "male meiosis cytokinesis",
  "gene_name": "Testicular spindle-associated protein SHCBP1L"
}